{
  "gene_symbol": "NLRC5",
  "term_label": "positive regulation of type II interferon-mediated signaling pathway",
  "term_id": "GO:0060335",
  "gene_name": "Protein NLRC5",
  "gene": "UniProtKB:Q86WI3"
}